{
  "term_label": "late endosome to Golgi transport",
  "gene_name": "Sorting nexin-12",
  "term_id": "GO:0034499",
  "gene": "UniProtKB:Q9UMY4",
  "gene_symbol": "SNX12"
}